cellular response to muramyl dipeptide [GO:0071225] (biological process) Definition: Any process that results in a change in state or activity of a cell (in terms of movement, secretion, enzyme production, gene expression, etc.) as a result of a muramyl dipeptide stimulus. Muramyl dipeptide is derived from peptidoglycan. Relationships: is_a response to muramyl dipeptide [GO:0032495]; is a type of GO:1901699; is a type of cellular response to oxygen-containing compound [GO:1901701] Sources: GOC:mah